{
  "gene": "UniProtKB:Q8NE18",
  "gene_symbol": "NSUN7",
  "term_id": "UNKNOWN:0002",
  "gene_name": "Putative methyltransferase NSUN7",
  "term_label": "Unknown biological process"
}